{
  "gene": "UniProtKB:Q9Y5P4",
  "term_label": "ceramide 1-phosphate binding",
  "gene_symbol": "CERT1",
  "term_id": "GO:1902387",
  "gene_name": "Ceramide transfer protein"
}